{
  "gene_name": "Transcription factor HES-2",
  "term_id": "GO:0000978",
  "term_label": "RNA polymerase II cis-regulatory region sequence-specific DNA binding",
  "gene_symbol": "HES2",
  "gene": "UniProtKB:Q9Y543"
}